{
  "gene": "UniProtKB:P26374",
  "gene_name": "Rab proteins geranylgeranyltransferase component A 2",
  "term_label": "cytosol",
  "gene_symbol": "CHML",
  "term_id": "GO:0005829"
}